{
  "term_label": "galactoside 2-alpha-L-fucosyltransferase activity",
  "gene": "UniProtKB:Q10981",
  "term_id": "GO:0008107",
  "gene_symbol": "FUT2",
  "gene_name": "Galactoside alpha-(1,2)-fucosyltransferase 2"
}